galactitol biosynthetic process [GO:0019403] (biological process) Sources: ISBN:0198506732 Relationships: is a type of galactitol metabolic process [GO:0019402]; is a type of hexitol biosynthetic process [GO:0019406] Also known as: galactitol anabolism, galactitol biosynthesis, galactitol formation, galactitol synthesis Definition: The chemical reactions and pathways resulting in the formation of galactitol, the hexitol derived by the reduction of the aldehyde group of either D- or L-galactose.